{
  "gene": "UniProtKB:P07478",
  "term_id": "GO:0004252",
  "gene_symbol": "PRSS2",
  "term_label": "serine-type endopeptidase activity",
  "gene_name": "Trypsin-2"
}